{
  "gene_symbol": "MANF",
  "term_label": "endoplasmic reticulum",
  "gene_name": "Mesencephalic astrocyte-derived neurotrophic factor",
  "term_id": "GO:0005783",
  "gene": "UniProtKB:P55145"
}